{
  "gene_name": "M-phase inducer phosphatase 3",
  "gene": "UniProtKB:P30307",
  "gene_symbol": "CDC25C",
  "term_id": "GO:0005737",
  "term_label": "cytoplasm"
}